{
  "term_id": "GO:0000213",
  "gene_name": "tRNA-splicing endonuclease subunit Sen2",
  "gene": "UniProtKB:Q8NCE0",
  "gene_symbol": "TSEN2",
  "term_label": "tRNA-intron lyase activity"
}